{
  "term_label": "olfactory receptor activity",
  "term_id": "GO:0004984",
  "gene": "UniProtKB:Q9H341",
  "gene_symbol": "OR51M1",
  "gene_name": "Olfactory receptor 51M1"
}